{
  "gene_symbol": "DXO",
  "term_label": "nuclear-transcribed mRNA catabolic process",
  "term_id": "GO:0000956",
  "gene_name": "Decapping and exoribonuclease protein",
  "gene": "UniProtKB:O77932"
}